regulation of basidiospore formation [GO:0075302] (biological process) Definition: Any process that modulates the frequency, rate or extent of basidiospore formation, a process in which a sexually produced fungal spore is formed on a basidium in the fungi Basidiomycetes. Subtypes: positive regulation of basidiospore formation [GO:0075303], negative regulation of basidiospore formation [GO:0075304] Sources: GOC:pamgo_curators Relationships: is a type of regulation of sexual sporulation resulting in formation of a cellular spore [GO:0043940]; regulates basidiospore formation [GO:0034295]